{
  "term_label": "smooth muscle cell differentiation",
  "gene": "UniProtKB:Q969V6",
  "gene_name": "Myocardin-related transcription factor A",
  "gene_symbol": "MRTFA",
  "term_id": "GO:0051145"
}